{
  "gene_symbol": "MRPL18",
  "term_id": "GO:0008097",
  "gene_name": "Large ribosomal subunit protein uL18m",
  "term_label": "5S rRNA binding",
  "gene": "UniProtKB:Q9H0U6"
}